protein phosphatase type 1 complex [GO:0000164] (cellular component) Subtypes: PTW/PP1 phosphatase complex [GO:0072357] Sources: GOC:mah, GOC:ssd Relationships: is a type of protein serine/threonine phosphatase complex [GO:0008287]; is part of cytoplasm [GO:0005737] Definition: A protein complex that possesses magnesium-dependent protein serine/threonine phosphatase (AMD phosphatase) activity, and consists of a catalytic subunit and one or more regulatory subunits that dictates the phosphatase's substrate specificity, function, and activity.